{
  "gene_name": "Peroxisomal membrane protein PMP34",
  "gene_symbol": "SLC25A17",
  "term_id": "GO:0005347",
  "gene": "UniProtKB:O43808",
  "term_label": "ATP transmembrane transporter activity"
}